{
  "gene": "UniProtKB:Q9UNM6",
  "term_id": "GO:0006511",
  "term_label": "ubiquitin-dependent protein catabolic process",
  "gene_symbol": "PSMD13",
  "gene_name": "26S proteasome non-ATPase regulatory subunit 13"
}